{
  "gene_symbol": "TAF6",
  "gene": "UniProtKB:P49848",
  "term_id": "GO:0016251",
  "gene_name": "Transcription initiation factor TFIID subunit 6",
  "term_label": "RNA polymerase II general transcription initiation factor activity"
}